{
  "gene_name": "Plasminogen receptor (KT)",
  "gene_symbol": "PLGRKT",
  "gene": "UniProtKB:Q9HBL7",
  "term_label": "positive regulation of plasminogen activation",
  "term_id": "GO:0010756"
}